regulation of monoatomic ion transport [GO:0043269] (biological process) Sources: GOC:jl Relationships: is a type of regulation of transport [GO:0051049]; regulates monoatomic ion transport [GO:0006811] Definition: Any process that modulates the frequency, rate or extent of the directed movement of charged atoms or small charged molecules into, out of or within a cell, or between cells, by means of some agent such as a transporter or pore. Also known as: regulation of ion transport Subtypes: GO:0010959, GO:0014062, regulation of monoatomic ion transmembrane transport [GO:0034765], positive regulation of monoatomic ion transport [GO:0043270], negative regulation of monoatomic ion transport [GO:0043271], GO:0044070